regulation of mannotriose transport [GO:1900327] (biological process) Sources: GOC:TermGenie, GOC:mengo_curators Definition: Any process that modulates the frequency, rate or extent of mannotriose transport. Subtypes: GO:1900328, positive regulation of mannotriose transport [GO:1900329] Relationships: is a type of GO:0051049; regulates mannotriose transport [GO:2001095]